{
  "term_id": "UNKNOWN:0003",
  "term_label": "Unknown cellular component",
  "gene_name": "Protein FAM106C",
  "gene": "UniProtKB:P0CH98",
  "gene_symbol": "FAM106C"
}